{
  "gene_name": "Bifunctional purine biosynthesis protein ATIC",
  "gene_symbol": "ATIC",
  "term_id": "GO:0003937",
  "term_label": "IMP cyclohydrolase activity",
  "gene": "UniProtKB:P31939"
}